tRNA (guanine(26)-N2)-dimethyltransferase activity [GO:0160104] (molecular function) Relationships: is a type of N-methyltransferase activity [GO:0008170]; is a type of GO:0016423 Also known as: tRNA (guanine(26)-N(2))-dimethyltransferase activity, tRNA (guanosine(26)-N(2))-dimethyltransferase activity, tRNA (m(2)2G26)dimethyltransferase Definition: Catalysis of the reaction:guanosine(26) in tRNA + 2 S-adenosyl-L-methionine = 2 H+ + N(2)-dimethylguanosine(26) in tRNA + 2 S-adenosyl-L-homocysteine. Sources: EC:2.1.1.216